{
  "gene_name": "Neuromedin-U receptor 2",
  "term_label": "neuropeptide signaling pathway",
  "gene": "UniProtKB:Q9GZQ4",
  "term_id": "GO:0007218",
  "gene_symbol": "NMUR2"
}